hydroxyphenylacetonitrile 2-monooxygenase activity [GO:0047085] (MF) Sources: RHEA:50732 Definition: Catalysis of the reaction: 4-hydroxyphenylacetonitrile + H+ + NADPH + O2 = 4-hydroxymandelonitrile + H2O + NADP+. Relationships: is a type of oxidoreductase activity, acting on paired donors, with incorporation or reduction of molecular oxygen, NAD(P)H as one donor, and incorporation of one atom of oxygen [GO:0016709] Also known as: 4-hydroxyphenylacetonitrile hydroxylase activity, 4-hydroxyphenylacetonitrile monooxygenase activity, 4-hydroxyphenylacetonitrile,NADPH:oxygen oxidoreductase (2-hydroxylating)